GABAergic neuron differentiation in basal ganglia [GO:0021858] (biological process) References: PMID:16226447 Sources: GOC:cls, GOC:dgh, GOC:dph, GOC:jid, GO_REF:0000021 Definition: The process in which a neuroblast acquires the specialized structural and functional features of a GABAergic inhibitory neuron in the basal ganglia. Differentiation includes the processes involved in commitment of a neuroblast to a GABAergic neuron. Relationships: is a type of GABAergic neuron differentiation [GO:0097154]